{
  "gene_symbol": "SOX11",
  "gene": "UniProtKB:P35716",
  "term_id": "GO:0030182",
  "gene_name": "Transcription factor SOX-11",
  "term_label": "neuron differentiation"
}